lysine biosynthetic process via alpha-aminoadipate and saccharopine [GO:0051975] (biological process) Sources: MetaCyc:LYSINE-AMINOAD-PWY Also known as: lysine biosynthesis via aminoadipic acid and saccharopine, lysine biosynthetic process via aminoadipic acid and saccharopine Regulation: regulated by regulation of lysine biosynthetic process via alpha-aminoadipate and saccharopine [GO:2001194]; negatively regulated by negative regulation of lysine biosynthetic process via alpha-aminoadipate and saccharopine [GO:2001195]; positively regulated by positive regulation of lysine biosynthetic process via alpha-aminoadipate and saccharopine [GO:2001196] Definition: The chemical reactions and pathways resulting in the formation of lysine via the intermediates alpha-aminoadipic acid and saccharopine. This pathway is used by yeast and fungi to synthesize the essential amino acid L-lysine, and pathway intermediates are often incorporated into secondary metabolic processes. The pathway proceeds as follows: alpha-ketoglutarate is converted to homocitrate, which is metabolized to 3-carboxyhex-2-enedioate and then homoisocitrate. This is then decarboxylated to form alpha-ketoadipate, which is then converted to alpha-aminoadipate. This is then reduced to form alpha-aminoadipate 6-semialdehyde, which is metabolized to saccharopine and finally L-lysine. Relationships: is a type of lysine biosynthetic process via aminoadipic acid [GO:0019878]